long-chain fatty acid omega-1 hydroxylase activity [GO:0120319] (molecular function) Definition: Catalysis of the reaction: an (omega-1)-ethyl long-chain fatty acid + O2 + reduced [NADPH-hemoprotein reductase] = an (omega-1)-hydroxy-long-chain fatty acid + H+ + H2O + oxidized [NADPH-hemoprotein reductase. A long-chain fatty acid has an aliphatic tail containing 13 to 22 carbons. Relationships: is a type of fatty acid omega-1 hydroxylase activity [GO:0120502] References: PMID:18577768, PMID:22772592, PMID:24242247 Sources: GOC:nhn, RHEA:60936 Note: While there is not universal consensus on the lengths of short-, medium-, long- and very-long-chain fatty acids, the GO uses the definitions in ChEBI (see CHEBI:26666, CHEBI:59554, CHEBI:15904 and CHEBI:27283). Also known as: cytochrome P450 fatty acid omega-1 hydroxylase activity